chromosome localization to nuclear envelope involved in homologous chromosome segregation [GO:0090220] (biological process) Definition: The directed movement of a chromosome to the nuclear envelope that contributes to homologous chromosome segregation and precedes synapsis. References: PMID:19913287 Sources: GOC:ascb_2009, GOC:dph, GOC:tb Also known as: chromosome localisation to nuclear envelope involved in homologous chromosome segregation Relationships: is a type of chromosome localization [GO:0050000]; BFO_0000050 homologous chromosome segregation [GO:0045143] Subtypes: meiotic telomere clustering [GO:0045141]